glyoxylate dehydrogenase (acylating) activity [GO:0047968] (molecular function) Also known as: glyoxylate:NADP+ oxidoreductase (CoA-oxalylating) Relationships: is a type of GO:0016620 Definition: Catalysis of the reaction: CoA + glyoxylate + NADP+ = H+ + NADPH + oxalyl-CoA. Sources: EC:1.2.1.17, RHEA:21024